{
  "gene_symbol": "RNASE10",
  "gene_name": "Inactive ribonuclease-like protein 10",
  "term_id": "UNKNOWN:0003",
  "term_label": "Unknown cellular component",
  "gene": "UniProtKB:Q5GAN6"
}